ectodermal placode development [GO:0071696] (biological process) Definition: The progression of an ectodermal placode over time from its initial formation until its mature state. An ectodermal placode is a thickening of the ectoderm that is the primordium of many structures derived from the ectoderm. Relationships: is_a GO:0048856 Sources: GOC:mah Subtypes: olfactory placode development [GO:0071698], otic placode development [GO:1905040]